DNA polymerase III, proofreading complex [GO:0043845] (cellular component) Definition: A subcomplex of DNA polymerase III composed of the epsilon subunit which has proofreading activity, and the theta subunit which enhances the epsilon subunit's proofreading activity. Also known as: DNA polymerase III, proof-reading complex, DNA polymerase III, proof-reading subcomplex, DNA polymerase III, proofreading subcomplex Relationships: is a type of GO:0140513; is part of GO:0044776 References: PMID:16973612 Sources: Wikipedia:Pol_III